{
  "gene": "UniProtKB:O14498",
  "term_label": "Unknown biological process",
  "gene_name": "Immunoglobulin superfamily containing leucine-rich repeat protein",
  "term_id": "UNKNOWN:0002",
  "gene_symbol": "ISLR"
}